{
  "term_label": "nucleus",
  "gene_symbol": "FIBP",
  "term_id": "GO:0005634",
  "gene": "UniProtKB:O43427",
  "gene_name": "Acidic fibroblast growth factor intracellular-binding protein"
}